{
  "gene": "UniProtKB:Q9UIF3",
  "term_label": "Unknown molecular function",
  "gene_name": "Tektin-2",
  "term_id": "UNKNOWN:0001",
  "gene_symbol": "TEKT2"
}